{
  "term_label": "immune response",
  "gene": "UniProtKB:P01704",
  "term_id": "GO:0006955",
  "gene_name": "Immunoglobulin lambda variable 2-14",
  "gene_symbol": "IGLV2-14"
}